{
  "gene_name": "Peroxisomal membrane protein 11C",
  "term_id": "UNKNOWN:0001",
  "gene_symbol": "PEX11G",
  "gene": "UniProtKB:Q96HA9",
  "term_label": "Unknown molecular function"
}